{
  "term_id": "GO:0016477",
  "gene_name": "Nck-associated protein 1-like",
  "gene_symbol": "NCKAP1L",
  "gene": "UniProtKB:P55160",
  "term_label": "cell migration"
}